{
  "gene_name": "Keratin, type I cuticular Ha1",
  "gene": "UniProtKB:Q15323",
  "term_id": "GO:0030280",
  "term_label": "structural constituent of skin epidermis",
  "gene_symbol": "KRT31"
}